{
  "gene_symbol": "UBE2J2",
  "term_label": "endoplasmic reticulum",
  "gene": "UniProtKB:Q8N2K1",
  "gene_name": "Ubiquitin-conjugating enzyme E2 J2",
  "term_id": "GO:0005783"
}